{
  "gene_symbol": "SRGAP2B",
  "gene_name": "SLIT-ROBO Rho GTPase-activating protein 2B",
  "term_id": "GO:0005096",
  "gene": "UniProtKB:P0DMP2",
  "term_label": "GTPase activator activity"
}